{
  "gene_symbol": "RBM44",
  "gene_name": "RNA-binding protein 44",
  "term_id": "GO:0003730",
  "term_label": "mRNA 3'-UTR binding",
  "gene": "UniProtKB:Q6ZP01"
}